detection of high humidity [GO:0098516] (biological process) Relationships: is a type of detection of humidity [GO:0098513] Sources: GOC:dos Subtypes: detection of high humidity stimulus involved in sensory perception [GO:0098514] Definition: The series of events in which high humidity is detected and converted into a molecular signal.